MHC class I protein complex [GO:0042612] (cellular component) Sources: GOC:add, GOC:jl, ISBN:0120781859, ISBN:0781735149 Definition: A transmembrane protein complex composed of a MHC class I alpha chain and an invariant beta2-microglobin chain, and with or without a bound peptide antigen. Class I here refers to classical class I molecules. Relationships: is a type of MHC protein complex [GO:0042611] Note: See also the cellular component term 'MHC class I peptide loading complex ; GO:0042824'.